{
  "term_id": "GO:0005794",
  "gene_symbol": "ZDHHC20",
  "gene_name": "Palmitoyltransferase ZDHHC20",
  "gene": "UniProtKB:Q5W0Z9",
  "term_label": "Golgi apparatus"
}